{
  "gene": "UniProtKB:Q9BXY0",
  "gene_name": "Protein MAK16 homolog",
  "term_label": "Unknown molecular function",
  "gene_symbol": "MAK16",
  "term_id": "UNKNOWN:0001"
}